{
  "term_label": "positive regulation of receptor signaling pathway via JAK-STAT",
  "gene_symbol": "PRL",
  "gene_name": "Prolactin",
  "term_id": "GO:0046427",
  "gene": "UniProtKB:P01236"
}